{
  "gene_symbol": "CYP39A1",
  "gene": "UniProtKB:Q9NYL5",
  "term_label": "cholesterol homeostasis",
  "term_id": "GO:0042632",
  "gene_name": "24-hydroxycholesterol 7-alpha-hydroxylase"
}